{
  "gene_symbol": "H2BC9",
  "term_id": "GO:0019731",
  "gene_name": "Histone H2B type 1-H",
  "gene": "UniProtKB:Q93079",
  "term_label": "antibacterial humoral response"
}